{
  "gene_name": "Protein salvador homolog 1",
  "term_id": "GO:0005829",
  "gene": "UniProtKB:Q9H4B6",
  "gene_symbol": "SAV1",
  "term_label": "cytosol"
}